{
  "gene_name": "Ubiquitin carboxyl-terminal hydrolase 37",
  "term_label": "G1/S transition of mitotic cell cycle",
  "term_id": "GO:0000082",
  "gene": "UniProtKB:Q86T82",
  "gene_symbol": "USP37"
}